establishment or maintenance of cytoskeleton polarity involved in ameboidal cell migration [GO:0003371] (biological process) Definition: Any cellular process that results in the specification, formation or maintenance of polarized cytoskeletal structures that contribute to the cell polarity of a migrating ameboid cell. Relationships: is a type of GO:0030952; is part of establishment of cell polarity involved in ameboidal cell migration [GO:0003365] Sources: GOC:ascb_2009, GOC:dph, GOC:tb Subtypes: GO:0003380